{
  "term_label": "Unknown cellular component",
  "term_id": "UNKNOWN:0003",
  "gene": "UniProtKB:Q9HBL7",
  "gene_name": "Plasminogen receptor (KT)",
  "gene_symbol": "PLGRKT"
}